post-embryonic hemopoiesis [GO:0035166] (biological process) Definition: The stages of blood cell formation that take place after completion of embryonic development. Sources: GOC:bf Also known as: post-embryonic haemopoiesis Relationships: is a type of hemopoiesis [GO:0030097]; is part of post-embryonic development [GO:0009791] Subtypes: larval lymph gland hemopoiesis [GO:0035167]